{
  "gene_name": "Protein odd-skipped-related 2",
  "term_id": "GO:0000122",
  "gene_symbol": "OSR2",
  "gene": "UniProtKB:Q8N2R0",
  "term_label": "negative regulation of transcription by RNA polymerase II"
}